tetrahydroxypteridine cycloisomerase activity [GO:0050329] (molecular function) Sources: EC:5.5.1.3, RHEA:18097 Definition: Catalysis of the reaction: tetrahydroxypteridine = H+ + xanthine-8-carboxylate. Relationships: is a type of GO:0016872 Also known as: tetrahydroxypteridine lyase (isomerizing)